{
  "term_id": "GO:0005794",
  "gene_name": "Ras-related protein Rab-10",
  "gene": "UniProtKB:P61026",
  "gene_symbol": "RAB10",
  "term_label": "Golgi apparatus"
}